{
  "gene": "UniProtKB:P40222",
  "gene_name": "Alpha-taxilin",
  "gene_symbol": "TXLNA",
  "term_id": "UNKNOWN:0003",
  "term_label": "Unknown cellular component"
}